{
  "gene_name": "Protein BEX4",
  "gene_symbol": "BEX4",
  "gene": "UniProtKB:Q9NWD9",
  "term_label": "Unknown molecular function",
  "term_id": "UNKNOWN:0001"
}